monoatomic ion-gated channel activity [GO:0022839] (molecular function) Definition: Enables the transmembrane transfer of a solute by a channel that opens in response to a specific ion stimulus. Subtypes: calcium-activated cation channel activity [GO:0005227], intracellular sodium-activated potassium channel activity [GO:0005228], chloride-activated potassium channel activity [GO:0070089] Relationships: is a type of GO:0022834 Also known as: ion gated channel activity, monoatomic ion gated channel activity Sources: GOC:mtg_transport